{
  "gene_symbol": "H1-0",
  "gene": "UniProtKB:P07305",
  "term_id": "GO:0030261",
  "term_label": "chromosome condensation",
  "gene_name": "Histone H1.0"
}